negative regulation of violaceol I biosynthetic process [GO:1900714] (biological process) Relationships: is a type of negative regulation of secondary metabolite biosynthetic process [GO:1900377]; is a type of regulation of violaceol I biosynthetic process [GO:1900713]; negatively regulates violaceol I biosynthetic process [GO:1900590] Sources: GOC:TermGenie, GOC:di Also known as: down regulation of violaceol I anabolism, down regulation of violaceol I biosynthesis, down regulation of violaceol I biosynthetic process, down regulation of violaceol I formation, down regulation of violaceol I synthesis, down-regulation of violaceol I anabolism, down-regulation of violaceol I biosynthesis, down-regulation of violaceol I biosynthetic process, down-regulation of violaceol I formation, down-regulation of violaceol I synthesis, downregulation of violaceol I anabolism, downregulation of violaceol I biosynthesis, downregulation of violaceol I biosynthetic process, downregulation of violaceol I formation, downregulation of violaceol I synthesis, inhibition of violaceol I anabolism, inhibition of violaceol I biosynthesis, inhibition of violaceol I formation, inhibition of violaceol I synthesis, negative regulation of violaceol I anabolism, negative regulation of violaceol I biosynthesis, negative regulation of violaceol I formation, negative regulation of violaceol I synthesis, inhibition of violaceol I biosynthetic process Definition: Any process that stops, prevents or reduces the frequency, rate or extent of violaceol I biosynthetic process.